{
  "term_label": "focal adhesion",
  "gene": "UniProtKB:Q8N8S7",
  "gene_symbol": "ENAH",
  "gene_name": "Protein enabled homolog",
  "term_id": "GO:0005925"
}